{
  "gene": "UniProtKB:Q8NEM1",
  "gene_name": "Zinc finger protein 680",
  "term_id": "GO:0006355",
  "gene_symbol": "ZNF680",
  "term_label": "regulation of DNA-templated transcription"
}